{
  "gene": "UniProtKB:Q9Y3Q3",
  "term_label": "endoplasmic reticulum",
  "gene_symbol": "TMED3",
  "gene_name": "Transmembrane emp24 domain-containing protein 3",
  "term_id": "GO:0005783"
}